{
  "term_id": "GO:0000278",
  "gene_name": "Tubulin beta-4B chain",
  "gene": "UniProtKB:P68371",
  "gene_symbol": "TUBB4B",
  "term_label": "mitotic cell cycle"
}